{
  "gene_symbol": "IL36B",
  "term_id": "GO:0005125",
  "gene": "UniProtKB:Q9NZH7",
  "gene_name": "Interleukin-36 beta",
  "term_label": "cytokine activity"
}